replication of extrachromosomal circular DNA [GO:0001326] (biological process) Relationships: is a type of DNA-templated DNA replication [GO:0006261] References: PMID:33867825 Sources: GOC:jh Definition: Replication of circular DNA following excision from the chromosome; replication of extrachromosomal circular DNA generally occurs independently of chromosomal replication.